{
  "gene_name": "Glutathione S-transferase A5",
  "gene_symbol": "GSTA5",
  "gene": "UniProtKB:Q7RTV2",
  "term_id": "GO:0006805",
  "term_label": "xenobiotic metabolic process"
}